{
  "gene": "UniProtKB:P78415",
  "gene_symbol": "IRX3",
  "term_label": "regulation of transcription by RNA polymerase II",
  "gene_name": "Iroquois-class homeodomain protein IRX-3",
  "term_id": "GO:0006357"
}